negative regulation of T cell differentiation in thymus [GO:0033085] (biological process) Sources: GOC:add, GOC:mah Also known as: negative regulation of thymic T cell differentiation, negative regulation of thymocyte cell differentiation, negative regulation of thymocyte differentiation, negative regulation of T cell development in thymus Relationships: is a type of regulation of T cell differentiation in thymus [GO:0033081]; is a type of negative regulation of T cell differentiation [GO:0045581]; negatively regulates GO:0033077 Subtypes: negative regulation of immature T cell proliferation in thymus [GO:0033088], negative regulation of positive thymic T cell selection [GO:1902233] Definition: Any process that stops, prevents, or reduces the frequency, rate or extent of T cell differentiation in the thymus. Note: Note that immunologists typically use the word 'development' to refer to cells of B or T cell lineages undergoing the process that GO describes as 'cell differentiation'.